{
  "gene_name": "Putative uncharacterized protein AFDN-DT",
  "term_id": "UNKNOWN:0001",
  "gene_symbol": "AFDN-DT",
  "gene": "UniProtKB:Q9Y6Z5",
  "term_label": "Unknown molecular function"
}